{
  "term_label": "SAM complex",
  "gene_symbol": "MTX2",
  "term_id": "GO:0001401",
  "gene": "UniProtKB:O75431",
  "gene_name": "Metaxin-2"
}